{
  "gene_name": "Triggering receptor expressed on myeloid cells 2",
  "term_label": "regulation of plasma membrane bounded cell projection organization",
  "gene_symbol": "TREM2",
  "gene": "UniProtKB:Q9NZC2",
  "term_id": "GO:0120035"
}